{
  "term_label": "Unknown molecular function",
  "gene_name": "Trichoplein keratin filament-binding protein",
  "gene_symbol": "TCHP",
  "gene": "UniProtKB:Q9BT92",
  "term_id": "UNKNOWN:0001"
}